excitation of vasomotor center by baroreceptor signaling [GO:0002010] (biological process) Definition: The process in which the molecular signal from the arterial baroreceptors is relayed to the vasomotor center causing it to signal increase arterial pressure. Also known as: excitation of vasomotor center by baroreceptor signalling Sources: GOC:dph Relationships: is a type of nervous system process involved in regulation of systemic arterial blood pressure [GO:0001976]; is part of baroreceptor response to decreased systemic arterial blood pressure [GO:0001982]